stem vascular tissue pattern formation [GO:0010222] (biological process) Definition: Vascular tissue pattern formation as it occurs in the stem of vascular plants. Sources: GOC:tb Relationships: is a type of GO:0010051